trans-Golgi network membrane [GO:0032588] (cellular component) Relationships: is a type of organelle membrane [GO:0031090]; is part of trans-Golgi network [GO:0005802] Also known as: trans Golgi network membrane, Golgi trans face membrane Definition: The lipid bilayer surrounding any of the compartments that make up the trans-Golgi network. Sources: GOC:mah